alphaE-beta7 integrin-E-cadherin complex [GO:0071064] (CC) Definition: A protein complex that consists of an alphaE-beta7 integrin complex bound to E-cadherin. References: PMID:10837471 Relationships: is a type of plasma membrane protein complex [GO:0098797] Also known as: ITGAE-ITGB7-CDH1 complex